RNA polymerase II complex binding [GO:0000993] (molecular function) Definition: Binding to an RNA polymerase II core enzyme, a multisubunit eukaryotic nuclear RNA polymerase typically composed of twelve subunits. Sources: GOC:txnOH Also known as: RNA polymerase II core binding, RNAP II core binding Relationships: is a type of basal RNA polymerase II transcription machinery binding [GO:0001099]; is a type of GO:0043175 Subtypes: RNA polymerase II complex recruiting activity [GO:0001139], RNA polymerase II C-terminal domain binding [GO:0099122]